{
  "term_label": "angiogenesis",
  "gene_name": "Apolipoprotein L domain-containing protein 1",
  "term_id": "GO:0001525",
  "gene": "UniProtKB:Q96LR9",
  "gene_symbol": "APOLD1"
}